oxidoreductase activity, acting on hydrogen as donor, NAD or NADP as acceptor [GO:0016696] (molecular function) Definition: Catalysis of an oxidation-reduction (redox) reaction in which hydrogen acts as an electron donor and reduces NAD or NADP. Sources: GOC:jl Relationships: is a type of oxidoreductase activity, acting on hydrogen as donor [GO:0016695] Subtypes: hydrogen dehydrogenase activity [GO:0047985], GO:0050583, hydrogenase activity (NAD+, ferredoxin) [GO:0102220]